{
  "gene": "UniProtKB:Q8TDQ1",
  "term_label": "plasma membrane",
  "term_id": "GO:0005886",
  "gene_name": "CMRF35-like molecule 1",
  "gene_symbol": "CD300LF"
}